{
  "gene_name": "UDP-N-acetylglucosamine transferase subunit ALG14 homolog",
  "gene": "UniProtKB:Q96F25",
  "gene_symbol": "ALG14",
  "term_id": "GO:0043541",
  "term_label": "UDP-N-acetylglucosamine transferase complex"
}